{
  "term_label": "Unknown biological process",
  "gene": "UniProtKB:Q9UBY9",
  "gene_symbol": "HSPB7",
  "gene_name": "Heat shock protein beta-7",
  "term_id": "UNKNOWN:0002"
}